female mating behavior [GO:0060180] (biological process) Sources: GOC:dph, GOC:pr, GOC:tb Definition: The specific behavior of a female organism that is associated with reproduction. Relationships: is a type of mating behavior [GO:0007617] Subtypes: female courtship behavior [GO:0008050], regulation of female receptivity [GO:0045924]